{
  "term_id": "UNKNOWN:0003",
  "gene_symbol": "LMO7DN",
  "gene_name": "LMO7 downstream neighbor protein",
  "gene": "UniProtKB:F2Z398",
  "term_label": "Unknown cellular component"
}